negative regulation of vesicle docking [GO:0106021] (biological process) Definition: Any process that stops, prevents, or reduces the frequency, rate or extent of vesicle docking. Relationships: is a type of GO:0048523; is a type of negative regulation of transport [GO:0051051]; is a type of regulation of vesicle docking [GO:0106020]; negatively regulates vesicle docking [GO:0048278] References: PMID:22810233 Also known as: negative regulation of vesicle to membrane docking